facial nerve formation [GO:0021611] (biological process) Definition: The process that gives rise to the facial nerve. This process pertains to the initial formation of a structure from unspecified parts. This sensory and motor nerve supplies the muscles of facial expression and the expression and taste at the anterior two-thirds of the tongue. The principal branches are the superficial ophthalmic, buccal, palatine and hyomandibular. The main trunk synapses within pterygopalatine ganglion in the parotid gland and this ganglion then gives of nerve branches which supply the lacrimal gland and the mucous secreting glands of the nasal and oral cavities. Also known as: CN VII biosynthesis, CN VII formation Relationships: is a type of cranial nerve formation [GO:0021603]; is part of facial nerve morphogenesis [GO:0021610] Sources: GOC:cls, GOC:dgh, GOC:dph, GOC:jid, GO_REF:0000021